isovaleryl-CoA(4-) catabolic process [GO:1902196] (biological process) Relationships: is a type of fatty-acyl-CoA catabolic process [GO:0036115] References: PMID:11231285 Sources: GOC:TermGenie Definition: The chemical reactions and pathways resulting in the breakdown of isovaleryl-CoA(4-). Also known as: isovaleryl-CoA(4-) breakdown, isovaleryl-CoA(4-) catabolism, isovaleryl-CoA(4-) degradation